{
  "gene_name": "von Willebrand factor",
  "gene": "UniProtKB:P04275",
  "term_label": "blood coagulation",
  "gene_symbol": "VWF",
  "term_id": "GO:0007596"
}